{
  "term_id": "GO:0006357",
  "term_label": "regulation of transcription by RNA polymerase II",
  "gene": "UniProtKB:Q9Y5R5",
  "gene_symbol": "DMRT2",
  "gene_name": "Doublesex- and mab-3-related transcription factor 2"
}